positive regulation of diacylglycerol biosynthetic process [GO:1900482] (biological process) Definition: Any process that activates or increases the frequency, rate or extent of diacylglycerol biosynthetic process. Sources: GOC:TermGenie Also known as: activation of diacylglycerol anabolism, activation of diacylglycerol biosynthesis, activation of diacylglycerol formation, activation of diacylglycerol synthesis, positive regulation of diacylglycerol anabolism, positive regulation of diacylglycerol biosynthesis, positive regulation of diacylglycerol formation, positive regulation of diacylglycerol synthesis, up regulation of diacylglycerol anabolism, up regulation of diacylglycerol biosynthesis, up regulation of diacylglycerol biosynthetic process, up regulation of diacylglycerol formation, up regulation of diacylglycerol synthesis, up-regulation of diacylglycerol anabolism, up-regulation of diacylglycerol biosynthesis, up-regulation of diacylglycerol biosynthetic process, up-regulation of diacylglycerol formation, up-regulation of diacylglycerol synthesis, upregulation of diacylglycerol anabolism, upregulation of diacylglycerol biosynthesis, upregulation of diacylglycerol biosynthetic process, upregulation of diacylglycerol formation, upregulation of diacylglycerol synthesis, activation of diacylglycerol biosynthetic process Relationships: is a type of positive regulation of lipid biosynthetic process [GO:0046889]; is a type of regulation of diacylglycerol biosynthetic process [GO:1900480]; positively regulates GO:0006651